{
  "gene_symbol": "NFU1",
  "term_id": "GO:0005739",
  "gene_name": "NFU1 iron-sulfur cluster scaffold homolog, mitochondrial",
  "gene": "UniProtKB:Q9UMS0",
  "term_label": "mitochondrion"
}